{
  "gene_name": "Striatin-interacting protein 1",
  "gene_symbol": "STRIP1",
  "term_label": "cytosol",
  "gene": "UniProtKB:Q5VSL9",
  "term_id": "GO:0005829"
}